{
  "term_id": "UNKNOWN:0003",
  "term_label": "Unknown cellular component",
  "gene_symbol": "A0A8V8TND5",
  "gene": "UniProtKB:A0A8V8TND5",
  "gene_name": "Uncharacterized protein"
}